{
  "term_id": "GO:0016567",
  "term_label": "protein ubiquitination",
  "gene_name": "Probable E3 ubiquitin-protein ligase HERC4",
  "gene": "UniProtKB:Q5GLZ8",
  "gene_symbol": "HERC4"
}